diacylglycerol-dependent, calcium-independent serine/threonine kinase activity [GO:0004699] (molecular function) Also known as: calcium-independent PKC activity, novel protein kinase C activity, atypical protein kinase C activity References: PMID:34834162 Definition: Catalysis of the reaction: ATP + a protein = ADP + a phosphoprotein. This reaction is activated by diacylglycerol but not by calcium. Relationships: is a type of diacylglycerol-dependent serine/threonine kinase activity [GO:0004697]